{
  "term_label": "DNA-binding transcription factor activity, RNA polymerase II-specific",
  "term_id": "GO:0000981",
  "gene_symbol": "STAT5A",
  "gene": "UniProtKB:P42229",
  "gene_name": "Signal transducer and activator of transcription 5A"
}